{
  "gene": "UniProtKB:Q9H0M5",
  "term_id": "GO:0000977",
  "gene_name": "Zinc finger protein 700",
  "term_label": "RNA polymerase II transcription regulatory region sequence-specific DNA binding",
  "gene_symbol": "ZNF700"
}